TTT Hsp90 cochaperone complex [GO:0110078] (CC) Also known as: TELO2-TTI1-TTI2, TTT complex, Tel2-Tti1-Tti2, Triple T complex Relationships: is_a protein-containing complex [GO:0032991] References: PMID:20810650, PMID:22505622, PMID:28827813, PMID:34233195 Definition: A Hsp90 cochaperone complex acting as an adapter between Hps90 and its substrates, members of the PIKK kinase family.